{
  "term_id": "GO:0006357",
  "term_label": "regulation of transcription by RNA polymerase II",
  "gene_name": "Zinc finger protein 564",
  "gene_symbol": "ZNF564",
  "gene": "UniProtKB:Q8TBZ8"
}